type I interferon receptor binding [GO:0005132] (molecular function) Relationships: is a type of cytokine receptor binding [GO:0005126]; is a type of GO:0044877 Definition: Binding to an interferon-type I receptor, a heterodimeric complex composed of an alpha subunit (IFNAR1) and a beta subunit (IFNAR2). References: PMID:17502368 Sources: GOC:ai, GOC:signaling Also known as: interferon-alpha/beta receptor binding, IFNAR1 binding, IFNAR2 binding, interferon-alpha/beta, interferon-alpha/beta receptor ligand, IFNAR binding